{
  "gene": "UniProtKB:Q9Y6H6",
  "gene_symbol": "KCNE3",
  "term_label": "delayed rectifier potassium channel activity",
  "term_id": "GO:0005251",
  "gene_name": "Potassium voltage-gated channel subfamily E member 3"
}